{
  "gene_name": "Potassium channel subfamily K member 2",
  "gene": "UniProtKB:O95069",
  "gene_symbol": "KCNK2",
  "term_label": "potassium ion transmembrane transport",
  "term_id": "GO:0071805"
}